symbiont-mediated suppression of host signal transduction pathway [GO:0052029] (biological process) Also known as: negative regulation by organism of signal transduction in other organism involved in symbiotic interaction, disruption by symbiont of host signal transduction pathway, disruption of host signal transduction pathway, down regulation by symbiont of host signal transduction pathway, down-regulation by symbiont of host signal transduction pathway, downregulation by symbiont of host signal transduction pathway, negative modulation by organism of host signal transduction pathway, negative regulation by symbiont of host signal transduction pathway, suppression by symbiont of host signal transduction pathway, inhibition by symbiont of host signal transduction pathway Sources: GOC:mtg_pamgo_17jul06 Subtypes: symbiont-mediated suppression of host JAK-STAT cascade [GO:0039514], symbiont-mediated suppression of host TRAF-mediated signal transduction [GO:0039527], symbiont-mediated suppression of host PKR/eIFalpha signaling [GO:0039580], symbiont-mediated suppression of host toll-like receptor signaling pathway [GO:0039722], symbiont-mediated suppression of host pathogen-associated molecular pattern receptor signaling pathway [GO:0052078], symbiont-mediated suppression of host G protein-coupled receptor signal transduction [GO:0075120], GO:0075135, symbiont-mediated suppression of host cAMP/PKA signal transduction [GO:0075210], symbiont-mediated suppression of host NF-kappaB cascade [GO:0085034], effector-mediated suppression of host salicylic acid-mediated innate immune signaling [GO:0140502], symbiont-mediated suppression of host interferon-mediated signaling pathway [GO:0140886], symbiont-mediated suppression of host MAPK cascade [GO:0141070], symbiont-mediated suppression of host tumor necrosis factor-mediated signaling pathway [GO:0141072], symbiont-mediated suppression of host signal transduction pathway via antagonism of host cell surface receptor [GO:0141129] Definition: A process in which a symbiont interferes with, inhibits or disrupts a host signal transduction pathway. The host is defined as the larger of the organisms involved in a symbiotic interaction. Relationships: is a type of symbiont-mediated perturbation of host signal transduction pathway [GO:0052027]